{
  "gene": "UniProtKB:O14862",
  "gene_symbol": "AIM2",
  "gene_name": "Interferon-inducible protein AIM2",
  "term_id": "GO:0005829",
  "term_label": "cytosol"
}